regulation of filamentous growth of a population of unicellular organisms in response to heat [GO:1900431] (biological process) Subtypes: negative regulation of filamentous growth of a population of unicellular organisms in response to heat [GO:1900432], positive regulation of filamentous growth of a population of unicellular organisms in response to heat [GO:1900433] Definition: Any process that modulates the frequency, rate or extent of filamentous growth of a population of unicellular organisms in response to heat. Relationships: is a type of regulation of response to stress [GO:0080134]; is a type of regulation of filamentous growth of a population of unicellular organisms [GO:1900428]; regulates filamentous growth of a population of unicellular organisms in response to heat [GO:0036168] Sources: GOC:TermGenie, GOC:di